{
  "gene_symbol": "DCAF12L1",
  "gene_name": "DDB1- and CUL4-associated factor 12-like protein 1",
  "term_label": "Cul4-RING E3 ubiquitin ligase complex",
  "term_id": "GO:0080008",
  "gene": "UniProtKB:Q5VU92"
}